{
  "term_label": "positive regulation of anterograde synaptic vesicle transport",
  "gene_symbol": "BORCS5",
  "term_id": "GO:1903744",
  "gene_name": "BLOC-1-related complex subunit 5",
  "gene": "UniProtKB:Q969J3"
}